{
  "term_label": "Unknown cellular component",
  "gene_symbol": "LRRC37A",
  "term_id": "UNKNOWN:0003",
  "gene_name": "Leucine-rich repeat-containing protein 37A",
  "gene": "UniProtKB:A6NMS7"
}